{
  "gene_name": "Uncharacterized protein C17orf114",
  "term_label": "Unknown biological process",
  "gene_symbol": "C17orf114",
  "term_id": "UNKNOWN:0002",
  "gene": "UniProtKB:A0A1B0GUV1"
}